{
  "gene": "UniProtKB:Q9NV64",
  "gene_symbol": "TMEM39A",
  "term_label": "negative regulation of autophagosome assembly",
  "term_id": "GO:1902902",
  "gene_name": "Transmembrane protein 39A"
}